{
  "gene_name": "Protein FAM90A27P",
  "gene_symbol": "FAM90A27P",
  "term_id": "UNKNOWN:0001",
  "gene": "UniProtKB:A6NNH2",
  "term_label": "Unknown molecular function"
}